{
  "gene": "UniProtKB:P02656",
  "gene_name": "Apolipoprotein C-III",
  "gene_symbol": "APOC3",
  "term_label": "spherical high-density lipoprotein particle",
  "term_id": "GO:0034366"
}